vesicle membrane [GO:0012506] (cellular component) Subtypes: cytoplasmic vesicle membrane [GO:0030659] Relationships: is a type of organelle membrane [GO:0031090]; is part of vesicle [GO:0031982] Sources: GOC:mah, GOC:vesicle Definition: The lipid bilayer surrounding any membrane-bounded vesicle in the cell.